{
  "term_id": "GO:0012506",
  "gene_symbol": "ANXA9",
  "gene_name": "Annexin A9",
  "gene": "UniProtKB:O76027",
  "term_label": "vesicle membrane"
}